xanthine dehydrogenase complex [GO:0002197] (cellular component) Definition: A homodimeric protein complex having xanthine dehydrogenase activity. Relationships: is a type of oxidoreductase complex [GO:1990204] References: PMID:8224915 Sources: GOC:hjd